{
  "gene_symbol": "PPIP5K1",
  "term_id": "GO:0000828",
  "gene_name": "Inositol hexakisphosphate and diphosphoinositol-pentakisphosphate kinase 1",
  "term_label": "inositol hexakisphosphate kinase activity",
  "gene": "UniProtKB:Q6PFW1"
}